{
  "gene_name": "Fanconi anemia group D2 protein",
  "gene": "UniProtKB:Q9BXW9",
  "term_label": "homologous chromosome pairing at meiosis",
  "gene_symbol": "FANCD2",
  "term_id": "GO:0007129"
}